{
  "term_id": "GO:0005096",
  "term_label": "GTPase activator activity",
  "gene": "UniProtKB:Q9NU19",
  "gene_symbol": "TBC1D22B",
  "gene_name": "TBC1 domain family member 22B"
}